{
  "gene_name": "Methyltransferase-like protein 22",
  "term_label": "protein methyltransferase activity",
  "gene": "UniProtKB:Q9BUU2",
  "gene_symbol": "METTL22",
  "term_id": "GO:0008276"
}